{
  "term_label": "Unknown cellular component",
  "gene": "UniProtKB:Q3LI72",
  "term_id": "UNKNOWN:0003",
  "gene_name": "Keratin-associated protein 19-5",
  "gene_symbol": "KRTAP19-5"
}